{
  "term_label": "modulation of chemical synaptic transmission",
  "term_id": "GO:0050804",
  "gene_symbol": "LRRC4",
  "gene_name": "Leucine-rich repeat-containing protein 4",
  "gene": "UniProtKB:Q9HBW1"
}